{
  "term_id": "GO:0016342",
  "gene_symbol": "CDH17",
  "gene_name": "Cadherin-17",
  "term_label": "catenin complex",
  "gene": "UniProtKB:Q12864"
}